6-phospho-beta-glucosidase activity [GO:0008706] (molecular function) Definition: Catalysis of the reaction: 6-phospho-beta-D-glucoside-(1,4)-D-glucose + H2O = D-glucose 6-phosphate + glucose. Sources: EC:3.2.1.86 Relationships: is a type of beta-glucosidase activity [GO:0008422] Also known as: 6-phospho-beta-D-glucosyl-(1,4)-D-glucose glucohydrolase activity, phospho-beta-glucosidase A, phospho-beta-glucosidase activity, phosphocellobiase activity